{
  "gene": "UniProtKB:Q12931",
  "gene_name": "Heat shock protein 75 kDa, mitochondrial",
  "term_id": "GO:0019901",
  "term_label": "protein kinase binding",
  "gene_symbol": "TRAP1"
}